{
  "term_id": "GO:0004568",
  "term_label": "chitinase activity",
  "gene_name": "Oviduct-specific glycoprotein",
  "gene_symbol": "OVGP1",
  "gene": "UniProtKB:Q12889"
}